regulation of fermentation [GO:0043465] (biological process) Subtypes: regulation of xylose catabolic process to ethanol [GO:1900515], GO:1901003, regulation of glucose catabolic process to lactate via pyruvate [GO:1904023] Definition: Any process that modulates the frequency, rate or extent of fermentation, the anaerobic enzymatic conversion of organic compounds, especially carbohydrates, to other compounds, especially to ethyl alcohol, resulting in energy in the form of adenosine triphosphate (ATP). Sources: GOC:jl Relationships: is a type of GO:0043467; RO_0002211 fermentation [GO:0006113]